{
  "gene_name": "Putative metallothionein MT1DP",
  "term_label": "cellular response to copper ion",
  "term_id": "GO:0071280",
  "gene_symbol": "MT1DP",
  "gene": "UniProtKB:A1L3X4"
}